{
  "term_label": "Unknown biological process",
  "gene_name": "Protein FAM117B",
  "gene": "UniProtKB:Q6P1L5",
  "term_id": "UNKNOWN:0002",
  "gene_symbol": "FAM117B"
}